{
  "term_label": "central nervous system development",
  "term_id": "GO:0007417",
  "gene_symbol": "SCIN",
  "gene": "UniProtKB:Q9Y6U3",
  "gene_name": "Scinderin"
}